{
  "gene": "UniProtKB:Q9NYY3",
  "gene_symbol": "PLK2",
  "term_id": "GO:0005814",
  "term_label": "centriole",
  "gene_name": "Serine_threonine-protein kinase PLK2"
}